{
  "term_label": "kainate selective glutamate receptor activity",
  "term_id": "GO:0015277",
  "gene": "UniProtKB:Q16099",
  "gene_name": "Glutamate receptor ionotropic, kainate 4",
  "gene_symbol": "GRIK4"
}